negative regulation of lamellipodium assembly [GO:0010593] (biological process) Definition: Any process that decreases the rate, frequency or extent of the formation of a lamellipodium, a thin sheetlike extension of the surface of a migrating cell. Relationships: is a type of regulation of lamellipodium assembly [GO:0010591]; is_a negative regulation of plasma membrane bounded cell projection assembly [GO:0120033]; is a type of negative regulation of lamellipodium organization [GO:1902744]; negatively regulates lamellipodium assembly [GO:0030032] Also known as: negative regulation of lamellipodium biogenesis Sources: GOC:dph, GOC:tb